box H/ACA scaRNP complex [GO:0072589] (cellular component) References: PMID:17284456, PMID:20227365 Sources: GOC:mah Also known as: nucleoplasmic box H/ACA RNP pseudouridylase complex Relationships: is a type of box H/ACA RNP complex [GO:0072588]; is a type of nuclear protein-containing complex [GO:0140513]; is a type of catalytic complex [GO:1902494]; is part of Cajal body [GO:0015030] Definition: A box H/ACA RNP complex that is located in the Cajal body of the nucleoplasm. In higher eukaryotes, box H/ACA RNP located in Cajal bodies mediate pseudouridylation of spliceosomal snRNAs.